{
  "term_id": "GO:0003735",
  "gene": "UniProtKB:P39023",
  "gene_symbol": "RPL3",
  "term_label": "structural constituent of ribosome",
  "gene_name": "Large ribosomal subunit protein uL3"
}